{
  "gene": "UniProtKB:Q9BSH3",
  "term_id": "UNKNOWN:0001",
  "term_label": "Unknown molecular function",
  "gene_symbol": "NICN1",
  "gene_name": "Nicolin-1"
}